{
  "gene_name": "Apolipoprotein A-I",
  "term_label": "high-density lipoprotein particle",
  "term_id": "GO:0034364",
  "gene_symbol": "APOA1",
  "gene": "UniProtKB:P02647"
}